{
  "term_id": "GO:0036089",
  "gene": "UniProtKB:Q8WWL2",
  "gene_name": "Protein spire homolog 2",
  "term_label": "cleavage furrow formation",
  "gene_symbol": "SPIRE2"
}